{
  "gene_name": "Protein transport protein Sec16B",
  "gene": "UniProtKB:Q96JE7",
  "term_id": "GO:0007029",
  "gene_symbol": "SEC16B",
  "term_label": "endoplasmic reticulum organization"
}